{
  "gene_name": "Beta-crystallin B1",
  "gene_symbol": "CRYBB1",
  "term_id": "UNKNOWN:0003",
  "gene": "UniProtKB:P53674",
  "term_label": "Unknown cellular component"
}